{
  "gene_name": "PP13850",
  "term_label": "Unknown molecular function",
  "term_id": "UNKNOWN:0001",
  "gene_symbol": "Q71RC1",
  "gene": "UniProtKB:Q71RC1"
}